positive regulation of compound eye retinal cell apoptotic process [GO:1901694] (biological process) Definition: Any process that activates or increases the frequency, rate or extent of compound eye retinal cell apoptotic process. Relationships: is a type of positive regulation of apoptotic process [GO:0043065]; is a type of positive regulation of compound eye retinal cell programmed cell death [GO:0046672]; is a type of regulation of compound eye retinal cell apoptotic process [GO:1901692]; positively regulates compound eye retinal cell apoptotic process [GO:1990010] References: PMID:12021768 Sources: GOC:TermGenie, GOC:mtg_apoptosis Also known as: up regulation of compound eye retinal cell apoptotic process, up-regulation of compound eye retinal cell apoptotic process, upregulation of compound eye retinal cell apoptotic process, activation of compound eye retinal cell apoptotic process, induction of compound eye retinal cell programmed cell death